voltage-gated calcium channel activity involved in AV node cell action potential [GO:0086056] (molecular function) Sources: GOC:BHF, GOC:mtg_cardiac_conduct_nov11 Relationships: is a type of voltage-gated calcium channel activity involved in cardiac muscle cell action potential [GO:0086007]; is part of membrane depolarization during AV node cell action potential [GO:0086045] Also known as: voltage-gated calcium channel activity involved in AV node cardiac muscle cell action potential, voltage-gated calcium channel activity involved in atrioventricular node cardiac muscle cell action potential Definition: Enables the transmembrane transfer of a calcium ion by a voltage-gated channel across the plasma membrane of an AV node cardiac muscle cell that contributes to the depolarization phase of an action potential. A voltage-gated channel is a channel whose open state is dependent on the voltage across the membrane in which it is embedded.